{
  "gene_name": "Mitochondrial carrier homolog 2",
  "term_id": "UNKNOWN:0001",
  "term_label": "Unknown molecular function",
  "gene": "UniProtKB:Q9Y6C9",
  "gene_symbol": "MTCH2"
}